{
  "gene": "UniProtKB:P52926",
  "gene_symbol": "HMGA2",
  "term_label": "transcription coregulator activity",
  "term_id": "GO:0003712",
  "gene_name": "High mobility group protein HMGI-C"
}